spermine acetylation [GO:0032919] (biological process) Definition: The modification of spermine by addition of acetyl groups. Relationships: is_a spermine metabolic process [GO:0008215]; is a type of GO:0032917 Sources: GOC:mlg